{
  "gene_symbol": "A0A8I5QJV6",
  "gene_name": "Uncharacterized protein",
  "term_id": "UNKNOWN:0002",
  "term_label": "Unknown biological process",
  "gene": "UniProtKB:A0A8I5QJV6"
}